{
  "gene": "UniProtKB:Q6ZSU1",
  "gene_symbol": "CYP2G1P",
  "gene_name": "Putative inactive cytochrome P450 2G1",
  "term_id": "UNKNOWN:0002",
  "term_label": "Unknown biological process"
}